{
  "gene": "UniProtKB:Q92688",
  "term_label": "regulation of apoptotic process",
  "gene_name": "Acidic leucine-rich nuclear phosphoprotein 32 family member B",
  "term_id": "GO:0042981",
  "gene_symbol": "ANP32B"
}